{
  "gene": "UniProtKB:Q99946",
  "term_id": "GO:0098978",
  "term_label": "glutamatergic synapse",
  "gene_name": "Proline-rich transmembrane protein 1",
  "gene_symbol": "PRRT1"
}